white fat cell proliferation [GO:0070343] (biological process) Definition: The multiplication or reproduction of white fat cells by cell division, resulting in the expansion of their population. Sources: CL:0000448, GOC:mah, GOC:sl Also known as: white adipocyte proliferation, white adipose cell proliferation Relationships: is a type of GO:0070341 Regulation: regulated by regulation of white fat cell proliferation [GO:0070350]; negatively regulated by GO:0070351; positively regulated by positive regulation of white fat cell proliferation [GO:0070352]